{
  "term_id": "GO:0006298",
  "gene_symbol": "PMS1",
  "gene_name": "PMS1 protein homolog 1",
  "gene": "UniProtKB:P54277",
  "term_label": "mismatch repair"
}